{
  "gene_symbol": "CDH2",
  "gene_name": "Cadherin-2",
  "gene": "UniProtKB:P19022",
  "term_id": "GO:0016339",
  "term_label": "calcium-dependent cell-cell adhesion"
}